{
  "gene_name": "Cyclin-dependent kinase 15",
  "gene_symbol": "CDK15",
  "term_label": "regulation of cell cycle phase transition",
  "term_id": "GO:1901987",
  "gene": "UniProtKB:Q96Q40"
}